{
  "gene": "UniProtKB:P21673",
  "gene_name": "Diamine acetyltransferase 1",
  "term_label": "spermidine acetylation",
  "gene_symbol": "SAT1",
  "term_id": "GO:0032918"
}